{
  "term_label": "prolyl-tRNA aminoacylation",
  "gene_name": "Bifunctional glutamate_proline--tRNA ligase",
  "gene": "UniProtKB:P07814",
  "gene_symbol": "EPRS1",
  "term_id": "GO:0006433"
}